Rel homology domain binding [GO:0044197] (molecular function) Definition: Binding to a Rel Homology Domain (RHD) of a protein. The RHD is found in a family of eukaryotic transcription factors, which includes NF-kappaB, Dorsal, Relish and NFAT. Also known as: RHD binding Sources: InterPro:IPR011539, Wikipedia:Rel_homology_domain Relationships: is a type of GO:0019904